{
  "gene_name": "Glutathione hydrolase light chain 2",
  "gene": "UniProtKB:Q14390",
  "term_label": "Unknown biological process",
  "term_id": "UNKNOWN:0002",
  "gene_symbol": "GGTLC2"
}